{
  "gene": "UniProtKB:Q15042",
  "term_label": "GTPase activator activity",
  "gene_symbol": "RAB3GAP1",
  "gene_name": "Rab3 GTPase-activating protein catalytic subunit",
  "term_id": "GO:0005096"
}